{
  "gene_name": "Transcription elongation factor A protein 3",
  "gene_symbol": "TCEA3",
  "term_label": "nucleus",
  "gene": "UniProtKB:O75764",
  "term_id": "GO:0005634"
}